{
  "term_id": "GO:0005634",
  "gene": "UniProtKB:Q9Y2T7",
  "gene_symbol": "YBX2",
  "gene_name": "Y-box-binding protein 2",
  "term_label": "nucleus"
}